{
  "gene": "UniProtKB:Q8N8E3",
  "term_label": "Unknown biological process",
  "term_id": "UNKNOWN:0002",
  "gene_name": "Centrosomal protein of 112 kDa",
  "gene_symbol": "CEP112"
}